establishment of planar polarity involved in nephron morphogenesis [GO:0072046] (biological process) Sources: GOC:mtg_kidney_jan10 Also known as: establishment of planar cell polarity involved in nephron morphogenesis Subtypes: establishment of planar polarity involved in mesonephric nephron morphogenesis [GO:0061238], establishment of planar polarity involved in metanephric nephron morphogenesis [GO:0072280] Relationships: is a type of establishment of planar polarity [GO:0001736]; is part of nephron morphogenesis [GO:0072028] Definition: Coordinated organization of groups of cells in the plane of an epithelium that contributes to the shaping of a nephron.